{
  "gene_symbol": "KCNJ2",
  "term_label": "Unknown molecular function",
  "gene_name": "Inward rectifier potassium channel 2",
  "term_id": "UNKNOWN:0001",
  "gene": "UniProtKB:P63252"
}